{
  "gene": "UniProtKB:Q07666",
  "term_id": "GO:0003729",
  "gene_symbol": "KHDRBS1",
  "term_label": "mRNA binding",
  "gene_name": "KH domain-containing, RNA-binding, signal transduction-associated protein 1"
}